{
  "gene_name": "Iron-sulfur protein NUBPL",
  "gene": "UniProtKB:Q8TB37",
  "term_id": "GO:0032981",
  "term_label": "mitochondrial respiratory chain complex I assembly",
  "gene_symbol": "NUBPL"
}